{
  "term_id": "GO:0045109",
  "term_label": "intermediate filament organization",
  "gene": "UniProtKB:Q2M2I5",
  "gene_symbol": "KRT24",
  "gene_name": "Keratin, type I cytoskeletal 24"
}